UDP-4-keto-rhamnose-4-keto-reductase activity [GO:0010490] (MF) Definition: Catalysis of the reaction: UDP-4-keto-rhamnose + NADPH = UDP-rhamnose + NADP+. References: PMID:17190829 Sources: GOC:tair_curators Relationships: is a type of oxidoreductase activity, acting on the CH-OH group of donors, NAD or NADP as acceptor [GO:0016616]